{
  "gene_name": "HAUS augmin-like complex subunit 4",
  "gene": "UniProtKB:Q9H6D7",
  "term_label": "spindle assembly",
  "gene_symbol": "HAUS4",
  "term_id": "GO:0051225"
}